{
  "gene_name": "Cilia- and flagella- associated protein 210",
  "gene_symbol": "CFAP210",
  "term_label": "Unknown biological process",
  "term_id": "UNKNOWN:0002",
  "gene": "UniProtKB:Q0VFZ6"
}